cellular response to humidity [GO:0071463] (biological process) Sources: GOC:mah Definition: Any process that results in a change in state or activity of a cell (in terms of movement, secretion, enzyme production, gene expression, etc.) as a result of a humidity stimulus, moisture in the atmosphere. Relationships: is a type of response to humidity [GO:0009270]; is a type of GO:0071462